{
  "term_id": "GO:0005525",
  "gene_name": "Tubulin alpha-4A chain",
  "gene": "UniProtKB:P68366",
  "gene_symbol": "TUBA4A",
  "term_label": "GTP binding"
}